{
  "gene_name": "E3 ubiquitin-protein ligase CCNB1IP1",
  "gene_symbol": "CCNB1IP1",
  "term_id": "UNKNOWN:0003",
  "gene": "UniProtKB:Q9NPC3",
  "term_label": "Unknown cellular component"
}